{
  "gene_symbol": "OVCH2",
  "term_label": "serine-type endopeptidase activity",
  "gene": "UniProtKB:Q7RTZ1",
  "gene_name": "Ovochymase-2",
  "term_id": "GO:0004252"
}